hydroxycinnamic acid transport [GO:1904952] (BP) References: PMID:26744218 Sources: GOC:TermGenie, GO_REF:0000065 Relationships: is a type of carboxylic acid transport [GO:0046942] Definition: The directed movement of a hydroxycinnamic acid into, out of or within a cell, or between cells, by means of some agent such as a transporter or pore.